{
  "gene": "UniProtKB:P23588",
  "gene_name": "Eukaryotic translation initiation factor 4B",
  "gene_symbol": "EIF4B",
  "term_label": "Unknown biological process",
  "term_id": "UNKNOWN:0002"
}